{
  "gene_symbol": "MYO3A",
  "term_id": "GO:0007605",
  "gene": "UniProtKB:Q8NEV4",
  "gene_name": "Myosin-IIIa",
  "term_label": "sensory perception of sound"
}